{
  "gene": "UniProtKB:P20794",
  "gene_name": "Serine_threonine-protein kinase MAK",
  "term_id": "GO:0060271",
  "term_label": "cilium assembly",
  "gene_symbol": "MAK"
}